Notch signaling pathway involved in arterial endothelial cell fate commitment [GO:0060853] (biological process) Relationships: is a type of Notch signaling pathway [GO:0007219]; is part of arterial endothelial cell fate commitment [GO:0060844] Also known as: Notch signalling pathway involved in arterial endothelial cell fate commitment Sources: GOC:dph, GOC:sdb_2009, GOC:tb Definition: The series of molecular signals initiated by binding of an extracellular ligand to a Notch receptor on the surface of the target cell and contributing to the commitment of a cell to an arterial endothelial cell fate.